{
  "gene_name": "Growth factor receptor-bound protein 2",
  "gene": "UniProtKB:P62993",
  "term_id": "GO:0005154",
  "gene_symbol": "GRB2",
  "term_label": "epidermal growth factor receptor binding"
}